{
  "term_id": "GO:0000981",
  "term_label": "DNA-binding transcription factor activity, RNA polymerase II-specific",
  "gene_symbol": "ZSCAN30",
  "gene_name": "Zinc finger and SCAN domain-containing protein 30",
  "gene": "UniProtKB:Q86W11"
}